ESCRT I complex [GO:0000813] (cellular component) Definition: An endosomal sorting complex required for transport. It consists of the class E vacuolar protein sorting (Vps) proteins and interacts with ubiquitinated cargoes. References: PMID:12892785, PMID:12900393 Sources: GOC:rb Also known as: endosomal sorting complex required for transport Relationships: is a type of ESCRT complex [GO:0036452]; is a type of membrane protein complex [GO:0098796]; is part of GO:0010008